{
  "term_id": "UNKNOWN:0002",
  "gene_symbol": "KLHDC3",
  "gene_name": "Kelch domain-containing protein 3",
  "term_label": "Unknown biological process",
  "gene": "UniProtKB:Q9BQ90"
}